{
  "term_id": "GO:0005874",
  "gene": "UniProtKB:Q86VH2",
  "term_label": "microtubule",
  "gene_name": "Kinesin-like protein KIF27",
  "gene_symbol": "KIF27"
}